{
  "gene_name": "StAR-related lipid transfer protein 6",
  "gene_symbol": "STARD6",
  "gene": "UniProtKB:P59095",
  "term_label": "Unknown biological process",
  "term_id": "UNKNOWN:0002"
}